U6 2'-O-snRNA methylation [GO:1990438] (biological process) Relationships: is a type of snRNA 2'-O-methylation [GO:1990437] Definition: The posttranscriptional addition a methyl group to the 2'-oxygen atom of a nucleotide residue in an U6 snRNA molecule. References: PMID:11842100, PMID:9844635